cyclic nucleotide-gated mechanosensitive monoatomic ion channel activity [GO:0043854] (molecular function) Also known as: cyclic nucleotide-gated mechanosensitive ion channel activity, cyclic nucleotide gated mechanosensitive ion channel activity, cyclic nucleotide regulated mechanosensitive ion channel, cyclic nucleotide-regulated mechanosensitive ion channel, small conductance mechanosensitive ion channel, MscS, cyclic nucleotide-regulated small mechanosensitive ion channel References: PMID:22206667 Sources: GOC:jl Definition: Enables the transmembrane transfer of an monoatomic ion by a channel that opens in response to a mechanical stress and when a cyclic nucleotide has been bound by the channel complex or one of its constituent parts. Relationships: is a type of mechanosensitive monoatomic ion channel activity [GO:0008381]